P2Y5 nucleotide receptor binding [GO:0031815] (molecular function) Definition: Binding to a P2Y5 nucleotide receptor. Also known as: P2Y5 nucleotide receptor ligand Sources: GOC:mah, GOC:nln Relationships: is_a G protein-coupled nucleotide receptor binding [GO:0031811]